{
  "gene": "UniProtKB:Q6PH85",
  "term_id": "GO:0031624",
  "gene_name": "DCN1-like protein 2",
  "gene_symbol": "DCUN1D2",
  "term_label": "ubiquitin conjugating enzyme binding"
}